demethylrebeccamycin--D-glucose O-methyltransferase activity [GO:0102082] (molecular function) Definition: Catalysis of the reaction: 4'-demethylrebeccamycin + S-adenosyl-L-methionine = H+ + rebeccamycin + S-adenosyl-L-homocysteine. Sources: EC:2.1.1.164, GOC:pz Relationships: is a type of methyltransferase activity [GO:0008168]